{
  "term_id": "GO:0019372",
  "gene_name": "Phospholipid hydroperoxide glutathione peroxidase",
  "term_label": "lipoxygenase pathway",
  "gene_symbol": "GPX4",
  "gene": "UniProtKB:P36969"
}